pullulan biosynthetic process [GO:0051677] (biological process) Sources: GOC:ai Definition: The chemical reactions and pathways resulting in the formation of pullulan, a neutral linear polysaccharide composed of repeating units of maltotriose joined by alpha-(1,6)-linkages. Relationships: is a type of GO:0009250; is a type of pullulan metabolic process [GO:0051676]